gastrin receptor activity [GO:0015054] (molecular function) Sources: GOC:ai, GOC:signaling Also known as: cholecystokinin-B receptor activity Relationships: is a type of G protein-coupled peptide receptor activity [GO:0008528] Definition: Combining with gastrin and transmitting the signal across the membrane by activating an associated G-protein to initiate a change in cell activity.